histone succinyltransferase activity [GO:0106078] (molecular function) Definition: Catalysis of the reaction: succinyl-CoA + histone = CoA + succinyl-histone. References: PMID:29211711 Relationships: is a type of peptide N-succinyltransferase activity [GO:0106075]; is a type of histone modifying activity [GO:0140993]